{
  "gene_name": "Integral membrane protein GPR137",
  "term_label": "negative regulation of bone resorption",
  "term_id": "GO:0045779",
  "gene": "UniProtKB:Q96N19",
  "gene_symbol": "GPR137"
}